{
  "term_label": "tRNA 5'-leader removal",
  "gene_name": "Ribonuclease P_MRP protein subunit POP5",
  "gene": "UniProtKB:Q969H6",
  "term_id": "GO:0001682",
  "gene_symbol": "POP5"
}